tetraketide alpha-pyrone synthase activity [GO:0090439] (molecular function) References: PMID:21193570 Sources: MetaCyc:RXN-16407 Relationships: is a type of acyltransferase activity, transferring groups other than amino-acyl groups [GO:0016747] Definition: Catalyzes the reaction: 7-hydroxylauroyl-CoA + 3 malonyl-CoA + 2 H+ = 2-(8-hydroxy-2-oxotridecyl)-6-oxopyran-4-olate + 3 CO2 + 4 coenzyme A.